dihydrolipoyllysine-residue acetyltransferase activity [GO:0004742] (MF) Definition: Catalysis of the reaction: N(6)-[(R)-dihydrolipoyl]-L-lysyl-[protein] + acetyl-CoA = N(6)-[(R)-S(8)-acetyldihydrolipoyl]-L-lysyl-[protein] + CoA. Sources: RHEA:17017 Also known as: dihydrolipoamide S-acetyltransferase activity, thioltransacetylase A activity, transacetylase X activity, acetyl-CoA: enzyme-6-N-(dihydrolipoyl)lysine S-acetyltransferase activity, acetyl-CoA: enzyme-N6-(dihydrolipoyl)lysine S-acetyltransferase activity, acetyl-CoA:dihydrolipoamide S-acetyltransferase activity, dihydrolipoamide S-acyltransferase activity, dihydrolipoate acetyltransferase activity, dihydrolipoic transacetylase activity, dihydrolipoyl acetyltransferase activity, enzyme-dihydrolipoyllysine:acetyl-CoA S-acetyltransferase activity, lipoate acetyltransferase activity, lipoate transacetylase activity, lipoic acetyltransferase activity, lipoic acid acetyltransferase activity, lipoic transacetylase activity, lipoylacetyltransferase activity Note: The only observed direction catalyzed by this activity is that where the acetyl group is passed to coenzyme A - that is, the right-to-left direction of that shown in the definition. Relationships: is a type of S-acetyltransferase activity [GO:0016418]; is a type of catalytic activity, acting on a protein [GO:0140096]